{
  "term_id": "UNKNOWN:0001",
  "gene_name": "EPM2A-interacting protein 1",
  "gene": "UniProtKB:Q7L775",
  "gene_symbol": "EPM2AIP1",
  "term_label": "Unknown molecular function"
}